negative regulation of inflammasome-mediated signaling pathway [GO:0141086] (biological process) References: PMID:33467177 Also known as: negative regulation of inflammasome-mediated signal transduction Relationships: is_a negative regulation of cytoplasmic pattern recognition receptor signaling pathway [GO:0039532]; is a type of regulation of inflammasome-mediated signaling pathway [GO:0141085]; negatively regulates inflammasome-mediated signaling pathway [GO:0141084] Definition: Any process that stops, prevents or reduces the frequency, rate or extent of an inflammasome-mediated signaling pathway.